{
  "gene": "UniProtKB:P38398",
  "gene_name": "Breast cancer type 1 susceptibility protein",
  "term_id": "GO:0031436",
  "gene_symbol": "BRCA1",
  "term_label": "BRCA1-BARD1 complex"
}